{
  "term_id": "UNKNOWN:0002",
  "gene_name": "Small ribosomal subunit protein mS22",
  "gene": "UniProtKB:P82650",
  "gene_symbol": "MRPS22",
  "term_label": "Unknown biological process"
}